{
  "term_label": "receptor antagonist activity",
  "gene_symbol": "WFIKKN1",
  "term_id": "GO:0048019",
  "gene_name": "WAP, Kazal, immunoglobulin, Kunitz and NTR domain-containing protein 1",
  "gene": "UniProtKB:Q96NZ8"
}